{
  "gene_name": "Diacylglycerol kinase kappa",
  "term_label": "diacylglycerol metabolic process",
  "gene": "UniProtKB:Q5KSL6",
  "term_id": "GO:0046339",
  "gene_symbol": "DGKK"
}